carbohydrate derivative binding [GO:0097367] (molecular function) Definition: Binding to a carbohydrate derivative. Subtypes: GO:0001530, nucleoside binding [GO:0001882], GO:0005539, GO:0008061, galactoside binding [GO:0016936], muramyl dipeptide binding [GO:0032500], deoxyribonucleotide binding [GO:0032552], ribonucleotide binding [GO:0032553], sialic acid binding [GO:0033691], lysophosphatidic acid binding [GO:0035727], proteoglycan binding [GO:0043394], GO:0046871, GO:0051861, fructose-6-phosphate binding [GO:0070095], GO:0070891, coenzyme F420 binding [GO:0070967], ADP-D-ribose binding [GO:0072570], poly-ADP-D-ribose binding [GO:0072572], glycosylated region protein binding [GO:0140081], 5-O-phosphono-alpha-D-ribofuranosyl diphosphate binding [GO:1902248], sn-glycerol 3-phosphate binding [GO:1902516], ascr#2 binding [GO:1904067], advanced glycation end-product binding [GO:1904599], lipooligosaccharide binding [GO:1990458], amylopectin binding [GO:2001066], beta-D-Gal-(1->4)-beta-D-GlcNAc-(1->3)-beta-D-Gal-(1->4)-D-Glc binding [GO:2001079], chitosan binding [GO:2001080], quercitrin binding [GO:2001227] Relationships: is a type of GO:0005488 Sources: GOC:pr